{
  "gene_symbol": "PPBP",
  "gene": "UniProtKB:P02775",
  "gene_name": "Platelet basic protein",
  "term_label": "cellular response to lipopolysaccharide",
  "term_id": "GO:0071222"
}